{
  "gene_symbol": "PTGFRN",
  "gene_name": "Prostaglandin F2 receptor negative regulator",
  "gene": "UniProtKB:Q9P2B2",
  "term_label": "Unknown biological process",
  "term_id": "UNKNOWN:0002"
}